{
  "gene_symbol": "DAPK2",
  "term_label": "protein serine/threonine kinase activity",
  "gene": "UniProtKB:Q9UIK4",
  "gene_name": "Death-associated protein kinase 2",
  "term_id": "GO:0004674"
}